{
  "gene": "UniProtKB:Q9GZY4",
  "term_id": "UNKNOWN:0001",
  "gene_name": "Cytochrome c oxidase assembly factor 1 homolog",
  "term_label": "Unknown molecular function",
  "gene_symbol": "COA1"
}